{
  "gene": "UniProtKB:Q9UKM9",
  "term_id": "UNKNOWN:0002",
  "gene_symbol": "RALY",
  "term_label": "Unknown biological process",
  "gene_name": "RNA-binding protein Raly"
}